{
  "gene_name": "Small ribosomal subunit protein eS12",
  "term_id": "GO:0003735",
  "gene_symbol": "RPS12",
  "gene": "UniProtKB:P25398",
  "term_label": "structural constituent of ribosome"
}